glycolytic process from glycerol [GO:0061613] (biological process) Sources: GOC:dph, ISBN:0201090910 Relationships: is_a glycolytic process [GO:0006096]; is a type of GO:0019563; has part triose-phosphate isomerase activity [GO:0004807]; has part GO:0061610 Definition: The glycolytic process in which glycerol is catabolized to pyruvate generating ATP and NADH.